{
  "term_label": "nucleus",
  "term_id": "GO:0005634",
  "gene_symbol": "ZNF418",
  "gene": "UniProtKB:Q8TF45",
  "gene_name": "Zinc finger protein 418"
}